{
  "gene_symbol": "NOL3",
  "term_id": "GO:2001243",
  "gene_name": "Nucleolar protein 3",
  "term_label": "negative regulation of intrinsic apoptotic signaling pathway",
  "gene": "UniProtKB:O60936"
}